{
  "gene_name": "Gamma-tubulin complex component 5",
  "gene_symbol": "TUBGCP5",
  "term_label": "mitotic cell cycle",
  "gene": "UniProtKB:Q96RT8",
  "term_id": "GO:0000278"
}